positive regulation of metaphase/anaphase transition of meiotic cell cycle [GO:1902104] (biological process) Also known as: activation of meiotic metaphase/anaphase transition, positive regulation of meiotic metaphase/anaphase transition, up regulation of meiotic metaphase/anaphase transition, up regulation of metaphase/anaphase transition of meiotic cell cycle, up-regulation of meiotic metaphase/anaphase transition, up-regulation of metaphase/anaphase transition of meiotic cell cycle, upregulation of meiotic metaphase/anaphase transition, upregulation of metaphase/anaphase transition of meiotic cell cycle, activation of metaphase/anaphase transition of meiotic cell cycle Relationships: is a type of GO:1901995; is a type of GO:1902101; is a type of regulation of metaphase/anaphase transition of meiotic cell cycle [GO:1902102]; is a type of positive regulation of meiotic chromosome separation [GO:1905134]; positively regulates metaphase/anaphase transition of meiotic cell cycle [GO:0044785] Definition: Any process that activates or increases the frequency, rate or extent of metaphase/anaphase transition of meiotic cell cycle. Sources: GOC:TermGenie, GOC:mtg_cell_cycle Subtypes: positive regulation of metaphase/anaphase transition of meiosis I [GO:1905188], GO:1905191